negative regulation of endocardial cushion cell differentiation [GO:0120076] (biological process) Definition: Any process that stops, prevents, or reduces the frequency, rate or extent of endocardial cushion cell differentiation. Sources: GOC:BHF, GOC:BHF_miRNA, GOC:rph Relationships: is a type of regulation of endocardial cushion cell differentiation [GO:0120074]; is a type of negative regulation of cardiocyte differentiation [GO:1905208]; negatively regulates endocardial cushion cell differentiation [GO:0061443]